{
  "gene_symbol": "OR5AR1",
  "term_label": "Unknown biological process",
  "term_id": "UNKNOWN:0002",
  "gene_name": "Olfactory receptor 5AR1",
  "gene": "UniProtKB:Q8NGP9"
}